D-glucose import [GO:0046323] (biological process) Definition: The directed movement of the hexose monosaccharide D-glucose into a cell or organelle. Subtypes: glucose import in response to insulin stimulus [GO:0044381] Sources: GOC:ai Relationships: is a type of D-glucose transmembrane transport [GO:1904659] Regulation: regulated by regulation of D-glucose import [GO:0046324]; negatively regulated by negative regulation of D-glucose import [GO:0046325]; positively regulated by positive regulation of D-glucose import [GO:0046326] Also known as: glucose import, glucose uptake